{
  "gene": "UniProtKB:Q12913",
  "gene_symbol": "PTPRJ",
  "gene_name": "Receptor-type tyrosine-protein phosphatase eta",
  "term_label": "signal transduction",
  "term_id": "GO:0007165"
}